{
  "term_label": "phosphatase activity",
  "gene_name": "Pseudouridine-5'-phosphatase",
  "term_id": "GO:0016791",
  "gene": "UniProtKB:Q08623",
  "gene_symbol": "PUDP"
}